{
  "term_id": "GO:0007204",
  "gene_name": "CAMPATH-1 antigen",
  "gene": "UniProtKB:P31358",
  "term_label": "positive regulation of cytosolic calcium ion concentration",
  "gene_symbol": "CD52"
}